{
  "gene_symbol": "PGM2L1",
  "term_id": "UNKNOWN:0003",
  "term_label": "Unknown cellular component",
  "gene_name": "Glucose 1,6-bisphosphate synthase",
  "gene": "UniProtKB:Q6PCE3"
}